{
  "gene": "UniProtKB:P51793",
  "gene_name": "H(+)_Cl(-) exchange transporter 4",
  "term_label": "plasma membrane",
  "gene_symbol": "CLCN4",
  "term_id": "GO:0005886"
}